{
  "gene_symbol": "OR11H1",
  "gene": "UniProtKB:Q8NG94",
  "term_id": "UNKNOWN:0002",
  "gene_name": "Olfactory receptor 11H1",
  "term_label": "Unknown biological process"
}